meiotic nuclear membrane disassembly [GO:0051078] (biological process) Definition: The cell cycle process in which the controlled breakdown of the nuclear membranes during meiotic cell division occurs. Sources: GOC:bf Also known as: meiotic nuclear envelope breakdown, meiotic nuclear envelope catabolism, meiotic nuclear envelope degradation, meiotic nuclear envelope disassembly Relationships: is a type of nuclear membrane disassembly [GO:0051081]; is_a meiotic cell cycle process [GO:1903046] Subtypes: meiosis I nuclear membrane disassembly [GO:0051079], meiosis II nuclear membrane disassembly [GO:0051080]